{
  "gene_name": "Angiopoietin-related protein 1",
  "gene_symbol": "ANGPTL1",
  "term_label": "signaling receptor binding",
  "term_id": "GO:0005102",
  "gene": "UniProtKB:O95841"
}